{
  "term_id": "GO:0071805",
  "term_label": "potassium ion transmembrane transport",
  "gene": "UniProtKB:Q4G0N8",
  "gene_name": "Sodium_hydrogen exchanger 10",
  "gene_symbol": "SLC9C1"
}